{
  "gene_name": "Acylamino-acid-releasing enzyme",
  "gene_symbol": "APEH",
  "term_id": "UNKNOWN:0002",
  "term_label": "Unknown biological process",
  "gene": "UniProtKB:P13798"
}